{
  "gene_symbol": "SYT9",
  "term_label": "calcium ion sensor activity",
  "gene_name": "Synaptotagmin-9",
  "gene": "UniProtKB:Q86SS6",
  "term_id": "GO:0061891"
}